{
  "gene_name": "CD180 antigen",
  "gene": "UniProtKB:Q99467",
  "gene_symbol": "CD180",
  "term_id": "GO:0038023",
  "term_label": "signaling receptor activity"
}